{
  "gene": "UniProtKB:A4FU28",
  "gene_name": "cTAGE family member 9",
  "term_id": "GO:0009306",
  "gene_symbol": "CTAGE9",
  "term_label": "protein secretion"
}